{
  "term_id": "GO:0005739",
  "gene": "UniProtKB:Q9H019",
  "term_label": "mitochondrion",
  "gene_name": "Mitochondrial fission regulator 1-like",
  "gene_symbol": "MTFR1L"
}